satellite DNA binding [GO:0003696] (molecular function) Relationships: is a type of sequence-specific double-stranded DNA binding [GO:1990837] Subtypes: microsatellite binding [GO:0035939] Sources: GOC:jl, SO:0000005 Definition: Binding to satellite DNA, the many tandem repeats (identical or related) of a short basic repeating unit; many have a base composition or other property different from the genome average that allows them to be separated from the bulk (main band) genomic DNA.